{
  "gene_symbol": "ZNF441",
  "gene_name": "Zinc finger protein 441",
  "gene": "UniProtKB:Q8N8Z8",
  "term_label": "DNA-binding transcription factor activity, RNA polymerase II-specific",
  "term_id": "GO:0000981"
}